{
  "gene_name": "Arfaptin-1",
  "term_label": "regulation of Arp2/3 complex-mediated actin nucleation",
  "term_id": "GO:0034315",
  "gene_symbol": "ARFIP1",
  "gene": "UniProtKB:P53367"
}